{
  "term_label": "glucuronosyltransferase activity",
  "term_id": "GO:0015020",
  "gene": "UniProtKB:O43505",
  "gene_name": "Beta-1,4-glucuronyltransferase 1",
  "gene_symbol": "B4GAT1"
}